{
  "term_id": "GO:0030291",
  "term_label": "protein serine/threonine kinase inhibitor activity",
  "gene": "UniProtKB:Q70Z35",
  "gene_name": "Phosphatidylinositol 3,4,5-trisphosphate-dependent Rac exchanger 2 protein",
  "gene_symbol": "PREX2"
}